{
  "term_label": "Unknown cellular component",
  "gene_name": "Beta-1,3-N-acetylglucosaminyltransferase lunatic fringe",
  "gene_symbol": "LFNG",
  "term_id": "UNKNOWN:0003",
  "gene": "UniProtKB:Q8NES3"
}